{
  "gene_name": "Histone H2A type 1-C",
  "term_label": "nucleosome",
  "gene_symbol": "H2AC6",
  "term_id": "GO:0000786",
  "gene": "UniProtKB:Q93077"
}